{
  "term_id": "UNKNOWN:0001",
  "gene_name": "Leucine-rich repeat and fibronectin type-III domain-containing protein 4",
  "term_label": "Unknown molecular function",
  "gene": "UniProtKB:Q6PJG9",
  "gene_symbol": "LRFN4"
}